histone H3K18ac reader activity [GO:0140044] (molecular function) Definition: A histone reader that recognizes a histone H3 acetylated at lysine 18. References: PMID:30110338 Also known as: histone H3K18ac modified histone binding Note: Comment: Note that the residue position corresponds to the canonical human H3 histone (UniProtKB:P84243); this residue is conserved across all eukaryotes. Residue 1 is the first residue following removal of the initiating Methionine (Met). Note that each histone is encoded by multiple genes, and sequences may vary across different genes within an organism. Relationships: is a type of GO:0140006